extrachromosomal circular DNA [GO:0005727] (cellular component) Sources: GOC:ai Subtypes: GO:0005728, 2-micrometer circle DNA [GO:0005729] Definition: Circular DNA structures that are not part of a chromosome. Relationships: is a type of intracellular anatomical structure [GO:0005622]; is part of extrachromosomal DNA [GO:0046821]